{
  "gene_symbol": "IRS4",
  "gene_name": "Insulin receptor substrate 4",
  "term_label": "insulin receptor binding",
  "gene": "UniProtKB:O14654",
  "term_id": "GO:0005158"
}